detection of maltose stimulus [GO:0034289] (biological process) Also known as: perception of maltose stimulus Sources: GOC:sart Relationships: is a type of response to maltose [GO:0034286]; is a type of GO:0034288 Definition: The series of events in which a maltose stimulus is received by a cell and converted into a molecular signal.